{
  "term_label": "Unknown molecular function",
  "gene_name": "Cytochrome c1, heme protein, mitochondrial",
  "gene": "UniProtKB:P08574",
  "term_id": "UNKNOWN:0001",
  "gene_symbol": "CYC1"
}